nicotine biosynthetic process [GO:0042179] (biological process) Relationships: is a type of GO:0009058; is a type of GO:0018933 Sources: GOC:sm, ISBN:0198547684 Definition: The chemical reactions and pathways resulting in the formation of nicotine, (S)(-)-3-(1-methyl-2-pyrrolidinyl)pyridine. Also known as: nicotine anabolism, nicotine biosynthesis, nicotine formation, nicotine synthesis